{
  "gene_symbol": "PCBD1",
  "term_label": "Unknown biological process",
  "gene_name": "Pterin-4-alpha-carbinolamine dehydratase",
  "term_id": "UNKNOWN:0002",
  "gene": "UniProtKB:P61457"
}